{
  "gene_name": "Olfactory receptor 8A1",
  "gene": "UniProtKB:Q8NGG7",
  "term_id": "GO:0005549",
  "gene_symbol": "OR8A1",
  "term_label": "odorant binding"
}